{
  "gene": "UniProtKB:Q8TF30",
  "term_label": "cytoplasm",
  "gene_name": "WASP homolog-associated protein with actin, membranes and microtubules",
  "gene_symbol": "WHAMM",
  "term_id": "GO:0005737"
}